{
  "gene_name": "Anaphase-promoting complex subunit 4",
  "gene": "UniProtKB:Q9UJX5",
  "gene_symbol": "ANAPC4",
  "term_id": "GO:0005680",
  "term_label": "anaphase-promoting complex"
}